{
  "term_label": "striated muscle tissue development",
  "gene": "UniProtKB:Q15124",
  "term_id": "GO:0014706",
  "gene_name": "Phosphoglucomutase-like protein 5",
  "gene_symbol": "PGM5"
}